{
  "gene": "UniProtKB:Q86VI4",
  "gene_symbol": "LAPTM4B",
  "term_label": "regulation of lysosomal membrane permeability",
  "term_id": "GO:0097213",
  "gene_name": "Lysosomal-associated transmembrane protein 4B"
}